{
  "gene_symbol": "U2AF1",
  "term_label": "spliceosomal complex",
  "gene_name": "Splicing factor U2AF 35 kDa subunit",
  "term_id": "GO:0005681",
  "gene": "UniProtKB:Q01081"
}